{
  "term_label": "vesicle fusion",
  "gene_symbol": "STX1A",
  "gene_name": "Syntaxin-1A",
  "term_id": "GO:0006906",
  "gene": "UniProtKB:Q16623"
}